{
  "gene_name": "Deoxyhypusine synthase",
  "gene": "UniProtKB:P49366",
  "term_label": "deoxyhypusine synthase activity",
  "term_id": "GO:0034038",
  "gene_symbol": "DHPS"
}